histone H4K16ac reader activity [GO:0140046] (molecular function) Definition: A histone reader that recognizes a histone H4 acetylated at lysine 16. References: PMID:16085498 Also known as: H4K16ac modified histone binding Note: Note that the residue position corresponds to the canonical human H4 histone (UniProtKB:P02309); this residue is conserved across all eukaryotes. Note that the initiation methionine is cleaved, so the first residue is S1. Relationships: is a type of histone H4 reader activity [GO:0140008]